{
  "gene": "UniProtKB:A0A075B6Z4",
  "gene_symbol": "TRDJ4",
  "gene_name": "T cell receptor delta joining 4 (Fragment)",
  "term_id": "UNKNOWN:0002",
  "term_label": "Unknown biological process"
}